{
  "gene": "UniProtKB:A0A6I8PU40",
  "term_label": "Unknown molecular function",
  "term_id": "UNKNOWN:0001",
  "gene_name": "Taurine up-regulated 1 protein",
  "gene_symbol": "TUG1"
}